{
  "term_id": "UNKNOWN:0001",
  "gene_name": "Transmembrane protein 256",
  "gene_symbol": "TMEM256",
  "gene": "UniProtKB:Q8N2U0",
  "term_label": "Unknown molecular function"
}